{
  "term_id": "GO:0000407",
  "gene": "UniProtKB:Q6PHR2",
  "gene_name": "Serine_threonine-protein kinase ULK3",
  "term_label": "phagophore assembly site",
  "gene_symbol": "ULK3"
}